{
  "gene_symbol": "DNM1L",
  "term_label": "microtubule binding",
  "gene_name": "Dynamin-1-like protein",
  "gene": "UniProtKB:O00429",
  "term_id": "GO:0008017"
}